response to hydroxyurea [GO:0072710] (biological process) Definition: Any process that results in a change in state or activity of a cell or an organism (in terms of movement, secretion, enzyme production, gene expression, etc.) as a result of a hydroxyurea stimulus. Relationships: is a type of response to nitrogen compound [GO:1901698] Sources: GOC:mah Also known as: response to HU Subtypes: cellular response to hydroxyurea [GO:0072711]